2-acylglycerol-3-phosphate O-acyltransferase activity [GO:0047144] (molecular function) Definition: Catalysis of the reaction: 2-acyl-sn-glycerol 3-phosphate + acyl-CoA = L-phosphatidate + CoA. Relationships: is a type of O-acyltransferase activity [GO:0008374]; is_a lysophosphatidic acid acyltransferase activity [GO:0042171] Sources: GOC:ab, RHEA:14233 Also known as: 2-acylglycerophosphate acyltransferase activity, acyl-CoA:2-acyl-sn-glycerol 3-phosphate O-acyltransferase activity